{
  "gene_symbol": "IGHV3-48",
  "gene_name": "Immunoglobulin heavy variable 3-48",
  "gene": "UniProtKB:P01763",
  "term_label": "Unknown cellular component",
  "term_id": "UNKNOWN:0003"
}